pantothenate transmembrane transporter activity [GO:0015233] (molecular function) Definition: Enables the directed movement of pantothenate across a membrane. Pantothenate is the anion of pantothenic acid, the amide of beta-alanine and pantoic acid; it is a B complex vitamin that is a constituent of coenzyme A and is distributed ubiquitously in foods. Sources: GOC:ai, ISBN:0721662544 Also known as: pantothenate transporter activity, vitamin B5 transmembrane transporter activity Relationships: is a type of amide transmembrane transporter activity [GO:0042887]; is a type of carboxylic acid transmembrane transporter activity [GO:0046943]; is a type of GO:0072349; is a type of GO:0090482; is part of pantothenate transmembrane transport [GO:0015887]